retinol O-fatty-acyltransferase activity [GO:0050252] (molecular function) Sources: EC:2.3.1.76, MetaCyc:RETINOL-O-FATTY-ACYLTRANSFERASE-RXN Also known as: acyl-CoA:retinol O-acyltransferase activity, retinol acyltransferase activity, retinol fatty-acyltransferase activity Relationships: is a type of O-acyltransferase activity [GO:0008374]; is part of retinol metabolic process [GO:0042572] Definition: Catalysis of the reaction: acyl-CoA + retinol = CoA + retinyl ester.